{
  "gene_name": "Taste receptor type 2 member 42",
  "gene_symbol": "TAS2R42",
  "term_label": "Unknown molecular function",
  "term_id": "UNKNOWN:0001",
  "gene": "UniProtKB:Q7RTR8"
}